{
  "gene_symbol": "HTR1E",
  "gene": "UniProtKB:P28566",
  "term_label": "neurotransmitter receptor activity",
  "gene_name": "5-hydroxytryptamine receptor 1E",
  "term_id": "GO:0030594"
}